{
  "term_label": "regulation of neurotransmitter secretion",
  "term_id": "GO:0046928",
  "gene_symbol": "MCTP2",
  "gene": "UniProtKB:Q6DN12",
  "gene_name": "Multiple C2 and transmembrane domain-containing protein 2"
}